{
  "term_id": "GO:0051607",
  "gene": "UniProtKB:P20592",
  "gene_symbol": "MX2",
  "term_label": "defense response to virus",
  "gene_name": "Interferon-induced GTP-binding protein Mx2"
}